{
  "term_label": "cytosol",
  "gene_symbol": "ABCE1",
  "gene": "UniProtKB:P61221",
  "term_id": "GO:0005829",
  "gene_name": "ATP-binding cassette sub-family E member 1"
}